{
  "term_id": "GO:0005184",
  "term_label": "neuropeptide hormone activity",
  "gene": "UniProtKB:P07492",
  "gene_name": "Gastrin-releasing peptide",
  "gene_symbol": "GRP"
}